{
  "gene": "UniProtKB:Q6PCB6",
  "gene_name": "Alpha_beta hydrolase domain-containing protein 17C",
  "term_id": "GO:0005886",
  "term_label": "plasma membrane",
  "gene_symbol": "ABHD17C"
}